{
  "term_id": "GO:0003735",
  "gene_symbol": "MRPL51",
  "term_label": "structural constituent of ribosome",
  "gene": "UniProtKB:Q4U2R6",
  "gene_name": "Large ribosomal subunit protein mL51"
}